{
  "term_id": "GO:0005794",
  "gene_name": "Ras-related protein Rab-6C",
  "term_label": "Golgi apparatus",
  "gene_symbol": "RAB6C",
  "gene": "UniProtKB:Q9H0N0"
}